{
  "term_label": "neuron projection",
  "term_id": "GO:0043005",
  "gene_symbol": "CADM1",
  "gene_name": "Cell adhesion molecule 1",
  "gene": "UniProtKB:Q9BY67"
}